negative regulation of cell size [GO:0045792] (BP) Also known as: down regulation of cell size, down-regulation of cell size, downregulation of cell size, inhibition of cell size Definition: Any process that reduces cell size. Relationships: is a type of regulation of cell size [GO:0008361] Sources: GOC:go_curators